meristem structural organization [GO:0009933] (biological process) Definition: Organization of a region of tissue in a plant that is composed of one or more undifferentiated cells capable of undergoing mitosis and differentiation, thereby effecting growth and development of a plant by giving rise to more meristem or specialized tissue. Also known as: meristem organisation, meristem organization Relationships: is a type of anatomical structure arrangement [GO:0048532]; is part of meristem development [GO:0048507] Regulation: regulated by regulation of meristem structural organization [GO:0009934] Sources: GOC:sm, ISBN:0198547684